{
  "term_label": "G protein-coupled receptor activity",
  "gene": "UniProtKB:Q86W33",
  "term_id": "GO:0004930",
  "gene_symbol": "TPRA1",
  "gene_name": "Transmembrane protein adipocyte-associated 1"
}